{
  "gene": "UniProtKB:O00329",
  "term_label": "plasma membrane",
  "gene_symbol": "PIK3CD",
  "gene_name": "Phosphatidylinositol 4,5-bisphosphate 3-kinase catalytic subunit delta isoform",
  "term_id": "GO:0005886"
}